{
  "term_id": "GO:0086100",
  "gene_symbol": "BCAR3",
  "gene_name": "Breast cancer anti-estrogen resistance protein 3",
  "term_label": "endothelin receptor signaling pathway",
  "gene": "UniProtKB:O75815"
}